detoxification of hydrogen peroxide [GO:0061691] (biological process) Relationships: is a type of GO:0042743; is a type of detoxification of inorganic compound [GO:0061687]; is part of response to hydrogen peroxide [GO:0042542] Sources: GOC:dph Subtypes: cellular detoxification of hydrogen peroxide [GO:0061692] Definition: Any process that reduces or removes the toxicity of hydrogen peroxide. These include transport of hydrogen peroxide away from sensitive areas and to compartments or complexes whose purpose is sequestration.